{
  "term_label": "canonical Wnt signaling pathway",
  "gene_name": "Frizzled-9",
  "gene": "UniProtKB:O00144",
  "term_id": "GO:0060070",
  "gene_symbol": "FZD9"
}